{
  "term_id": "UNKNOWN:0001",
  "term_label": "Unknown molecular function",
  "gene_name": "Transmembrane protein 150A",
  "gene_symbol": "TMEM150A",
  "gene": "UniProtKB:Q86TG1"
}